{
  "gene": "UniProtKB:Q15257",
  "term_id": "GO:0005737",
  "gene_symbol": "PTPA",
  "term_label": "cytoplasm",
  "gene_name": "Serine_threonine-protein phosphatase 2A activator"
}